{
  "gene": "UniProtKB:P01584",
  "gene_symbol": "IL1B",
  "gene_name": "Interleukin-1 beta",
  "term_id": "GO:0071222",
  "term_label": "cellular response to lipopolysaccharide"
}